{
  "term_id": "UNKNOWN:0002",
  "gene": "UniProtKB:P60903",
  "gene_symbol": "S100A10",
  "term_label": "Unknown biological process",
  "gene_name": "Protein S100-A10"
}